{
  "gene": "UniProtKB:Q5HY92",
  "term_label": "ATP hydrolysis activity",
  "gene_name": "Fidgetin",
  "gene_symbol": "FIGN",
  "term_id": "GO:0016887"
}